{
  "gene_symbol": "METTL25",
  "gene": "UniProtKB:Q8N6Q8",
  "term_id": "UNKNOWN:0001",
  "term_label": "Unknown molecular function",
  "gene_name": "Probable methyltransferase-like protein 25"
}